{
  "term_label": "Unknown biological process",
  "term_id": "UNKNOWN:0002",
  "gene_symbol": "MPRIP",
  "gene": "UniProtKB:Q6WCQ1",
  "gene_name": "Myosin phosphatase Rho-interacting protein"
}